{
  "gene_name": "Activin receptor type-1",
  "term_label": "BMP signaling pathway",
  "term_id": "GO:0030509",
  "gene": "UniProtKB:Q04771",
  "gene_symbol": "ACVR1"
}